DNA damage response, signal transduction resulting in transcription [GO:0042772] (biological process) Sources: GOC:go_curators Relationships: is_a signal transduction in response to DNA damage [GO:0042770] Definition: A cascade of processes initiated in response to the detection of DNA damage, and resulting in the induction of transcription.